{
  "term_id": "GO:0019902",
  "gene_name": "Short transient receptor potential channel 4-associated protein",
  "gene": "UniProtKB:Q8TEL6",
  "term_label": "phosphatase binding",
  "gene_symbol": "TRPC4AP"
}